{
  "term_id": "GO:0005615",
  "gene": "UniProtKB:Q9Y251",
  "gene_symbol": "HPSE",
  "term_label": "extracellular space",
  "gene_name": "Heparanase"
}